{
  "gene_symbol": "MYL2",
  "gene": "UniProtKB:P10916",
  "term_label": "muscle cell fate specification",
  "gene_name": "Myosin regulatory light chain 2, ventricular_cardiac muscle isoform",
  "term_id": "GO:0042694"
}